{
  "term_label": "Unknown biological process",
  "term_id": "UNKNOWN:0002",
  "gene_name": "ADAMTS-like protein 1",
  "gene": "UniProtKB:Q8N6G6",
  "gene_symbol": "ADAMTSL1"
}